{
  "gene_symbol": "COX11",
  "term_id": "UNKNOWN:0001",
  "gene_name": "Cytochrome c oxidase assembly protein COX11, mitochondrial",
  "term_label": "Unknown molecular function",
  "gene": "UniProtKB:Q9Y6N1"
}